{
  "gene_name": "Zinc finger protein 740",
  "gene": "UniProtKB:Q8NDX6",
  "gene_symbol": "ZNF740",
  "term_id": "GO:0006357",
  "term_label": "regulation of transcription by RNA polymerase II"
}